{
  "term_label": "nucleus",
  "gene_name": "G protein-coupled receptor associated sorting protein 3",
  "gene_symbol": "GPRASP3",
  "gene": "UniProtKB:Q6PI77",
  "term_id": "GO:0005634"
}